{
  "gene_symbol": "CCDC167",
  "term_id": "UNKNOWN:0002",
  "gene": "UniProtKB:Q9P0B6",
  "gene_name": "Coiled-coil domain-containing protein 167",
  "term_label": "Unknown biological process"
}